{
  "gene_symbol": "NUDT10",
  "gene_name": "Diphosphoinositol polyphosphate phosphohydrolase 3-alpha",
  "term_label": "diadenosine hexaphosphate catabolic process",
  "gene": "UniProtKB:Q8NFP7",
  "term_id": "GO:1901909"
}